inositol hexakisphosphate 3-phosphatase activity [GO:0016158] (molecular function) Relationships: is a type of GO:0004446 Also known as: phytase activity, 3-phytase activity, myo-inositol-hexaphosphate 3-phosphohydrolase activity, phytate 3-phosphatase activity, 1-phytase activity, myo-inositol-hexakisphosphate 3-phosphohydrolase activity, phytate 1-phosphatase activity Sources: EC:3.1.3.8 Definition: Catalysis of the reaction: myo-inositol hexakisphosphate + H2O = D-myo-inositol 1,2,4,5,6-pentakisphosphate + phosphate.